{
  "gene_symbol": "CD6",
  "term_id": "GO:0005886",
  "term_label": "plasma membrane",
  "gene_name": "T-cell differentiation antigen CD6",
  "gene": "UniProtKB:P30203"
}